response to vitamin A [GO:0033189] (biological process) Subtypes: GO:0071299 Definition: Any process that results in a change in state or activity of a cell or an organism (in terms of movement, secretion, enzyme production, gene expression, etc.) as a result of a vitamin A stimulus. Relationships: is a type of response to vitamin [GO:0033273]; is a type of GO:0033993 Sources: GOC:sl Also known as: response to retinol